positive regulation of retrograde dense core granule transport [GO:1901956] (BP) Relationships: is a type of positive regulation of vesicle transport along microtubule [GO:1901610]; is_a GO:1901954; is a type of positive regulation of dense core granule transport [GO:1904811]; is a type of GO:2001019; positively regulates GO:1990049 References: PMID:23358451 Sources: GOC:TermGenie, GOC:kmv Definition: Any process that activates or increases the frequency, rate or extent of retrograde dense core granule transport. Also known as: up regulation of retrograde dense core granule transport, up-regulation of retrograde dense core granule transport, upregulation of retrograde dense core granule transport, activation of retrograde dense core granule transport